regulation of glutamate uptake involved in transmission of nerve impulse [GO:0051946] (biological process) Also known as: regulation of L-glutamate reuptake, regulation of L-glutamate uptake during transmission of nerve impulse, regulation of glutamate reuptake, regulation of glutamate uptake involved in conduction of nerve impulse, regulation of glutamate uptake during transmission of nerve impulse Definition: Any process that modulates the frequency, rate or extent of the directed movement of L-glutamate into a neuron or glial cell. Subtypes: GO:0051948, positive regulation of glutamate uptake involved in transmission of nerve impulse [GO:0051951] Sources: GOC:ai Relationships: is a type of regulation of L-glutamate import across plasma membrane [GO:0002036]; is_a GO:0051941; regulates glutamate reuptake [GO:0051935]